{
  "term_id": "GO:1905515",
  "term_label": "non-motile cilium assembly",
  "gene_name": "Transmembrane protein 107",
  "gene": "UniProtKB:Q6UX40",
  "gene_symbol": "TMEM107"
}